adenohypophysis formation [GO:0048847] (biological process) Definition: The process that gives rise to adenohypophysis. This process pertains to the initial formation of a structure from unspecified parts. The adenohypophysis is the anterior part of the pituitary. It secretes a variety of hormones and its function is regulated by the hypothalamus. Sources: GOC:cvs, GOC:dgh, GOC:dph, GOC:jid Also known as: adenophysis biosynthesis, adenophysis formation, anterior pituitary biosynthesis, anterior pituitary formation, anterior pituitary gland biosynthesis, anterior pituitary gland formation Relationships: is a type of anatomical structure formation involved in morphogenesis [GO:0048646]; is part of adenohypophysis morphogenesis [GO:0048855]